{
  "term_label": "olfactory receptor activity",
  "gene": "UniProtKB:Q8NH01",
  "gene_symbol": "OR2T11",
  "gene_name": "Olfactory receptor 2T11",
  "term_id": "GO:0004984"
}